{
  "term_id": "GO:0005886",
  "gene_symbol": "SLC4A11",
  "gene": "UniProtKB:Q8NBS3",
  "term_label": "plasma membrane",
  "gene_name": "Solute carrier family 4 member 11"
}